{
  "gene": "UniProtKB:Q5TF39",
  "gene_name": "Sodium-dependent glucose transporter 1",
  "term_label": "Unknown biological process",
  "gene_symbol": "MFSD4B",
  "term_id": "UNKNOWN:0002"
}